{
  "gene": "UniProtKB:Q9P2V4",
  "term_label": "Unknown biological process",
  "term_id": "UNKNOWN:0002",
  "gene_symbol": "LRIT1",
  "gene_name": "Leucine-rich repeat, immunoglobulin-like domain and transmembrane domain-containing protein 1"
}